{
  "gene_name": "NHL repeat-containing protein 2",
  "term_id": "UNKNOWN:0003",
  "term_label": "Unknown cellular component",
  "gene": "UniProtKB:Q8NBF2",
  "gene_symbol": "NHLRC2"
}